{
  "gene_name": "A-kinase anchor protein 4",
  "term_label": "sperm fibrous sheath",
  "gene_symbol": "AKAP4",
  "term_id": "GO:0035686",
  "gene": "UniProtKB:Q5JQC9"
}